{
  "gene_name": "Potassium voltage-gated channel subfamily KQT member 1",
  "term_label": "voltage-gated potassium channel complex",
  "gene": "UniProtKB:P51787",
  "term_id": "GO:0008076",
  "gene_symbol": "KCNQ1"
}